{
  "gene_name": "EF-hand calcium-binding domain-containing protein 12",
  "gene_symbol": "EFCAB12",
  "term_label": "Unknown biological process",
  "gene": "UniProtKB:Q6NXP0",
  "term_id": "UNKNOWN:0002"
}